methane catabolic process [GO:0046188] (biological process) Sources: GOC:ai Also known as: methane breakdown, methane catabolism, methane degradation Relationships: is a type of methane metabolic process [GO:0015947]; is a type of GO:0043448 Definition: The chemical reactions and pathways resulting in the breakdown of methane, a colorless, odorless, flammable gas with the formula CH4. It is the simplest of the alkanes.